{
  "gene": "UniProtKB:A2PYH4",
  "gene_name": "Probable ATP-dependent DNA helicase HFM1",
  "term_label": "resolution of meiotic recombination intermediates",
  "gene_symbol": "HFM1",
  "term_id": "GO:0000712"
}